{
  "gene": "UniProtKB:Q0VDE8",
  "term_id": "GO:0050872",
  "term_label": "white fat cell differentiation",
  "gene_symbol": "ADIG",
  "gene_name": "Adipogenin"
}